{
  "term_label": "DNA-binding transcription factor activity, RNA polymerase II-specific",
  "gene_symbol": "ZSCAN32",
  "gene_name": "Zinc finger and SCAN domain-containing protein 32",
  "gene": "UniProtKB:Q9NX65",
  "term_id": "GO:0000981"
}